{
  "gene_name": "VPS9 domain-containing protein 1",
  "term_label": "small GTPase binding",
  "term_id": "GO:0031267",
  "gene_symbol": "VPS9D1",
  "gene": "UniProtKB:Q9Y2B5"
}